{
  "gene_symbol": "ENPP4",
  "term_label": "Unknown cellular component",
  "gene": "UniProtKB:Q9Y6X5",
  "term_id": "UNKNOWN:0003",
  "gene_name": "Bis(5'-adenosyl)-triphosphatase ENPP4"
}